{
  "gene_name": "E3 ubiquitin-protein ligase makorin-1",
  "gene_symbol": "MKRN1",
  "gene": "UniProtKB:Q9UHC7",
  "term_id": "GO:0061630",
  "term_label": "ubiquitin protein ligase activity"
}